cleavage furrow [GO:0032154] (cellular component) Relationships: is a type of plasma membrane region [GO:0098590]; is part of cell division site [GO:0032153] Definition: The cleavage furrow is a plasma membrane invagination at the cell division site. The cleavage furrow begins as a shallow groove and eventually deepens to divide the cytoplasm. Sources: GOC:vw, ISBN:0805319409 Note: While the term 'cleavage furrow' was initially associated with animal cells, such a structure occurs in many other types of cells, including unicellular protists.